{
  "term_id": "GO:0016139",
  "term_label": "glycoside catabolic process",
  "gene": "UniProtKB:Q9BTY2",
  "gene_symbol": "FUCA2",
  "gene_name": "Plasma alpha-L-fucosidase"
}